{
  "term_id": "UNKNOWN:0003",
  "gene": "UniProtKB:Q6IPX1",
  "term_label": "Unknown cellular component",
  "gene_symbol": "TBC1D3C",
  "gene_name": "TBC1 domain family member 3C"
}